{
  "gene": "UniProtKB:Q99447",
  "gene_name": "Ethanolamine-phosphate cytidylyltransferase",
  "gene_symbol": "PCYT2",
  "term_id": "GO:0005737",
  "term_label": "cytoplasm"
}